{
  "term_label": "nucleus",
  "term_id": "GO:0005634",
  "gene_name": "Cyclin-dependent kinase 18",
  "gene_symbol": "CDK18",
  "gene": "UniProtKB:Q07002"
}